{
  "gene": "UniProtKB:O00482",
  "term_label": "hormone-mediated signaling pathway",
  "term_id": "GO:0009755",
  "gene_name": "Nuclear receptor subfamily 5 group A member 2",
  "gene_symbol": "NR5A2"
}